uracil catabolic process [GO:0006212] (biological process) Relationships: is a type of GO:0006208; is a type of uracil metabolic process [GO:0019860] Definition: The chemical reactions and pathways resulting in the breakdown of uracil, 2,4-dioxopyrimidine, one of the pyrimidine bases occurring in RNA, but not in DNA. Sources: GOC:go_curators Also known as: uracil breakdown, uracil catabolism, uracil degradation